{
  "term_label": "gap junction channel activity",
  "gene_symbol": "GJD4",
  "gene_name": "Gap junction delta-4 protein",
  "gene": "UniProtKB:Q96KN9",
  "term_id": "GO:0005243"
}